{
  "term_id": "GO:0005096",
  "gene_name": "Rho GTPase-activating protein 6",
  "gene": "UniProtKB:O43182",
  "term_label": "GTPase activator activity",
  "gene_symbol": "ARHGAP6"
}